{
  "gene_symbol": "ANXA2R",
  "term_label": "Unknown biological process",
  "term_id": "UNKNOWN:0002",
  "gene_name": "Annexin-2 receptor",
  "gene": "UniProtKB:Q3ZCQ2"
}